{
  "gene": "UniProtKB:P29034",
  "term_label": "endothelial cell migration",
  "gene_name": "Protein S100-A2",
  "gene_symbol": "S100A2",
  "term_id": "GO:0043542"
}